inositol trisphosphate metabolic process [GO:0032957] (biological process) Also known as: IP3 metabolic process, IP3 metabolism, inositol trisphosphate metabolism, myo-inositol trisphosphate metabolic process Sources: GOC:mah Relationships: is a type of GO:0043647 Subtypes: inositol trisphosphate biosynthetic process [GO:0032959] Definition: The chemical reactions and pathways involving myo-inositol phosphate, 1,2,3,4,5,6-cyclohexanehexol, with three phosphate groups attached.